{
  "gene": "UniProtKB:Q08AM6",
  "gene_name": "Protein VAC14 homolog",
  "term_label": "endosome membrane",
  "term_id": "GO:0010008",
  "gene_symbol": "VAC14"
}